courtship behavior [GO:0007619] (biological process) Sources: GOC:ai, GOC:dph Subtypes: male courtship behavior [GO:0008049], GO:0008050 Relationships: is a type of mating behavior [GO:0007617] Definition: The behavior of an organism for the purpose of attracting sexual partners. Also known as: courtship behaviour